{
  "gene_name": "Fibroblast growth factor 5",
  "term_label": "extracellular space",
  "gene": "UniProtKB:P12034",
  "gene_symbol": "FGF5",
  "term_id": "GO:0005615"
}